{
  "term_label": "response to selenium ion",
  "gene": "UniProtKB:P07203",
  "gene_symbol": "GPX1",
  "term_id": "GO:0010269",
  "gene_name": "Glutathione peroxidase 1"
}